{
  "term_label": "protein stabilization",
  "gene_name": "E3 ubiquitin-protein ligase TRIM39",
  "gene": "UniProtKB:Q9HCM9",
  "term_id": "GO:0050821",
  "gene_symbol": "TRIM39"
}